{
  "gene_name": "Secretoglobin family 2B member 2",
  "term_label": "Unknown molecular function",
  "term_id": "UNKNOWN:0001",
  "gene_symbol": "SCGB2B2",
  "gene": "UniProtKB:Q4G0G5"
}